{
  "gene_name": "Nicotinamide_nicotinic acid mononucleotide adenylyltransferase 2",
  "term_label": "nicotinate-nucleotide adenylyltransferase activity",
  "gene_symbol": "NMNAT2",
  "term_id": "GO:0004515",
  "gene": "UniProtKB:Q9BZQ4"
}